{
  "gene_name": "Zinc finger protein GLIS3",
  "term_id": "GO:0000978",
  "gene": "UniProtKB:Q8NEA6",
  "term_label": "RNA polymerase II cis-regulatory region sequence-specific DNA binding",
  "gene_symbol": "GLIS3"
}